{
  "gene": "UniProtKB:O00555",
  "term_id": "GO:0005891",
  "gene_symbol": "CACNA1A",
  "gene_name": "Voltage-dependent P_Q-type calcium channel subunit alpha-1A",
  "term_label": "voltage-gated calcium channel complex"
}